intercellular transport [GO:0010496] (biological process) Relationships: is a type of transport [GO:0006810]; is a type of GO:0009987 Sources: GOC:dhl Definition: The movement of substances between cells. Subtypes: plasmodesmata-mediated intercellular transport [GO:0010497], vesicle-mediated intercellular transport [GO:0110077], gap junction-mediated intercellular transport [GO:1990349] Also known as: single organism intercellular transport, single-organism intercellular transport